response to molecule of oomycetes origin [GO:0002240] (biological process) Subtypes: detection of molecule of oomycetes origin [GO:0032492], cellular response to molecule of oomycetes origin [GO:0071227] Definition: Any process that results in a change in state or activity of an organism (in terms of movement, secretion, enzyme production, gene expression, etc.) as a result of a stimulus by molecules of oomycetes origin. Also known as: response to oomycetes associated molecule Sources: GOC:rl, GOC:sm Relationships: is a type of response to external biotic stimulus [GO:0043207]; is part of response to oomycetes [GO:0002239]